regulation of phosphatidylinositol 3-kinase/protein kinase B signal transduction [GO:0051896] (BP) Relationships: is a type of GO:1902531; regulates phosphatidylinositol 3-kinase/protein kinase B signal transduction [GO:0043491] Sources: GOC:ai Definition: Any process that modulates the frequency, rate or extent of phosphatidylinositol 3-kinase/protein kinase B signal transduction. Also known as: regulation of PI3K-PKB/Akt pathway, regulation of PI3K/Akt signal transduction, regulation of PI3K/PKB signal transduction, regulation of phosphatidylinositol 3-kinase signaling/protein kinase B signal transduction, regulation of AKT signaling cascade, regulation of AKT signalling cascade, regulation of PKB signaling cascade, regulation of PKB signalling cascade, regulation of protein kinase B signaling, regulation of protein kinase B signaling cascade, regulation of protein kinase B signalling cascade Subtypes: positive regulation of phosphatidylinositol 3-kinase/protein kinase B signal transduction [GO:0051897], negative regulation of phosphatidylinositol 3-kinase/protein kinase B signal transduction [GO:0051898]